negative regulation of F-9775A biosynthetic process [GO:1900671] (biological process) Definition: Any process that stops, prevents or reduces the frequency, rate or extent of F-9775A biosynthetic process. Sources: GOC:TermGenie, GOC:di Relationships: is a type of regulation of F-9775A biosynthetic process [GO:1900670]; is_a negative regulation of polyketide biosynthetic process [GO:1900733]; negatively regulates GO:1900611 Also known as: down regulation of F-9775A anabolism, down regulation of F-9775A biosynthesis, down regulation of F-9775A biosynthetic process, down regulation of F-9775A formation, down regulation of F-9775A synthesis, down-regulation of F-9775A anabolism, down-regulation of F-9775A biosynthesis, down-regulation of F-9775A biosynthetic process, down-regulation of F-9775A formation, down-regulation of F-9775A synthesis, downregulation of F-9775A anabolism, downregulation of F-9775A biosynthesis, downregulation of F-9775A biosynthetic process, downregulation of F-9775A formation, downregulation of F-9775A synthesis, inhibition of F-9775A anabolism, inhibition of F-9775A biosynthesis, inhibition of F-9775A formation, inhibition of F-9775A synthesis, negative regulation of F-9775A anabolism, negative regulation of F-9775A biosynthesis, negative regulation of F-9775A formation, negative regulation of F-9775A synthesis, inhibition of F-9775A biosynthetic process